{
  "gene_symbol": "ZDHHC12",
  "term_id": "GO:0019706",
  "gene": "UniProtKB:Q96GR4",
  "gene_name": "Palmitoyltransferase ZDHHC12",
  "term_label": "protein-cysteine S-palmitoyltransferase activity"
}